development of secondary male sexual characteristics [GO:0046544] (biological process) Definition: The process whose specific outcome is the progression of the secondary male sexual characteristics over time, from their formation to the mature structures. In male humans, these include growth of axillary, chest, and pubic hair, voice changes, and testicular/penile enlargement. Development occurs in response to sex hormone secretion. Sources: GOC:ai Relationships: is_a development of secondary sexual characteristics [GO:0045136]; is part of male sex differentiation [GO:0046661]